{
  "term_label": "positive regulation of transcription by RNA polymerase II",
  "gene_name": "Nuclear receptor-interacting protein 1",
  "gene": "UniProtKB:P48552",
  "gene_symbol": "NRIP1",
  "term_id": "GO:0045944"
}